{
  "term_id": "GO:0005154",
  "gene_name": "Epigen",
  "term_label": "epidermal growth factor receptor binding",
  "gene": "UniProtKB:Q6UW88",
  "gene_symbol": "EPGN"
}